{
  "gene": "UniProtKB:Q8N8Y2",
  "term_label": "plasma membrane proton-transporting V-type ATPase complex",
  "gene_symbol": "ATP6V0D2",
  "gene_name": "V-type proton ATPase subunit d 2",
  "term_id": "GO:0033181"
}